{
  "gene": "UniProtKB:P04141",
  "term_id": "GO:0030099",
  "gene_symbol": "CSF2",
  "gene_name": "Granulocyte-macrophage colony-stimulating factor",
  "term_label": "myeloid cell differentiation"
}